{
  "term_label": "extracellular space",
  "term_id": "GO:0005615",
  "gene": "UniProtKB:P04628",
  "gene_name": "Proto-oncogene Wnt-1",
  "gene_symbol": "WNT1"
}